positive regulation of phosphatidylcholine biosynthetic process [GO:2001247] (biological process) Also known as: positive regulation of phosphatidylcholine anabolism, positive regulation of phosphatidylcholine biosynthesis, positive regulation of phosphatidylcholine formation, positive regulation of phosphatidylcholine synthesis Relationships: is a type of positive regulation of phospholipid biosynthetic process [GO:0071073]; is a type of regulation of phosphatidylcholine biosynthetic process [GO:2001245]; positively regulates phosphatidylcholine biosynthetic process [GO:0006656] Sources: GOC:obol Definition: Any process that activates or increases the frequency, rate or extent of phosphatidylcholine biosynthetic process.